{
  "gene": "UniProtKB:Q6PH85",
  "gene_name": "DCN1-like protein 2",
  "term_label": "protein neddylation",
  "gene_symbol": "DCUN1D2",
  "term_id": "GO:0045116"
}